clathrin-sculpted acetylcholine transport vesicle [GO:0060200] (CC) Also known as: clathrin sculpted acetylcholine constitutive secretory pathway transport vesicle, clathrin sculpted acetylcholine transport vesicle Definition: A clathrin-sculpted lipid bilayer membrane-enclosed vesicle after clathrin release and containing acetylcholine. Sources: GOC:dph Relationships: is a type of transport vesicle [GO:0030133]; is a type of clathrin-sculpted vesicle [GO:0060198]